{
  "gene": "UniProtKB:P01909",
  "term_id": "GO:0042613",
  "term_label": "MHC class II protein complex",
  "gene_symbol": "HLA-DQA1",
  "gene_name": "HLA class II histocompatibility antigen, DQ alpha 1 chain"
}